positive regulation of type III hypersensitivity [GO:0001805] (biological process) Sources: GOC:add, ISBN:0781735149 Relationships: is a type of regulation of type III hypersensitivity [GO:0001803]; is a type of GO:0002885; is a type of positive regulation of myeloid leukocyte mediated immunity [GO:0002888]; is a type of positive regulation of immunoglobulin mediated immune response [GO:0002891]; positively regulates type III hypersensitivity [GO:0001802] Also known as: up regulation of type III hypersensitivity, up-regulation of type III hypersensitivity, upregulation of type III hypersensitivity, activation of type III hypersensitivity, stimulation of type III hypersensitivity Definition: Any process that activates or increases the frequency, rate or extent of type III hypersensitivity, a type of inflammatory response.